{
  "gene_name": "PTB-containing, cubilin and LRP1-interacting protein",
  "term_id": "GO:2000377",
  "gene": "UniProtKB:Q7Z2X4",
  "gene_symbol": "PID1",
  "term_label": "regulation of reactive oxygen species metabolic process"
}